{
  "term_id": "GO:0031519",
  "gene": "UniProtKB:Q96MM3",
  "term_label": "PcG protein complex",
  "gene_symbol": "ZFP42",
  "gene_name": "Zinc finger protein 42 homolog"
}